interferon regulatory factor 3-interferon regulatory factor 7 complex [GO:0097075] (cellular component) Definition: An interferon regulatory factor complex that consists of a heterodimer of interferon regulatory factor 3 and interferon regulatory factor 7. References: PMID:18068231 Sources: GOC:cna Also known as: IRF3:IRF7 complex Relationships: is a type of interferon regulatory factor complex [GO:0097071]